{
  "gene_symbol": "FLRT2",
  "term_id": "GO:0005615",
  "gene_name": "Leucine-rich repeat transmembrane protein FLRT2",
  "gene": "UniProtKB:O43155",
  "term_label": "extracellular space"
}